{
  "gene": "UniProtKB:Q4G0S4",
  "term_id": "GO:0005739",
  "term_label": "mitochondrion",
  "gene_symbol": "CYP27C1",
  "gene_name": "Cytochrome P450 27C1"
}